{
  "term_label": "potassium ion homeostasis",
  "term_id": "GO:0055075",
  "gene_name": "Solute carrier family 12 member 7",
  "gene_symbol": "SLC12A7",
  "gene": "UniProtKB:Q9Y666"
}